{
  "gene": "UniProtKB:Q9H8Q6",
  "gene_symbol": "HEXA-AS1",
  "term_label": "Unknown molecular function",
  "gene_name": "Putative uncharacterized protein encoded by HEXA-AS1",
  "term_id": "UNKNOWN:0001"
}